{
  "gene": "UniProtKB:Q9H3R0",
  "gene_name": "Lysine-specific demethylase 4C",
  "term_id": "GO:0005634",
  "gene_symbol": "KDM4C",
  "term_label": "nucleus"
}